{
  "term_id": "GO:0032880",
  "gene_symbol": "GHRH",
  "term_label": "regulation of protein localization",
  "gene": "UniProtKB:P01286",
  "gene_name": "Somatoliberin"
}